{
  "term_label": "serine-type peptidase activity",
  "gene_symbol": "PRSS51",
  "term_id": "GO:0008236",
  "gene_name": "Serine protease-like protein 51",
  "gene": "UniProtKB:A0A1B0GVH4"
}